locomotion [GO:0040011] (biological process) Relationships: is a type of biological_process [GO:0008150] Regulation: regulated by GO:0040012; negatively regulated by negative regulation of locomotion [GO:0040013]; positively regulated by GO:0040017 Definition: Self-propelled movement of a cell or organism from one location to another. Sources: GOC:dgh Subtypes: locomotion involved in locomotory behavior [GO:0031987], directional locomotion [GO:0033058], swimming [GO:0036268], taxis [GO:0042330], flight [GO:0060361], GO:0071965